{
  "gene": "UniProtKB:P12644",
  "gene_name": "Bone morphogenetic protein 4",
  "term_label": "cytokine activity",
  "gene_symbol": "BMP4",
  "term_id": "GO:0005125"
}